{
  "gene_name": "SAM and SH3 domain-containing protein 1",
  "term_id": "GO:0031435",
  "gene_symbol": "SASH1",
  "gene": "UniProtKB:O94885",
  "term_label": "mitogen-activated protein kinase kinase kinase binding"
}